{
  "gene_symbol": "REEP2",
  "gene_name": "Receptor expression-enhancing protein 2",
  "term_id": "GO:0008017",
  "gene": "UniProtKB:Q9BRK0",
  "term_label": "microtubule binding"
}